{
  "gene_name": "Monocarboxylate transporter 1",
  "gene": "UniProtKB:P53985",
  "gene_symbol": "SLC16A1",
  "term_label": "plasma membrane",
  "term_id": "GO:0005886"
}